membrane depolarization during Purkinje myocyte cell action potential [GO:0086047] (biological process) Relationships: is a type of membrane depolarization during cardiac muscle cell action potential [GO:0086012]; is part of GO:0086017 Sources: GOC:BHF, GOC:mtg_cardiac_conduct_nov11 Definition: The process in which Purkinje myocyte membrane potential changes in the depolarizing direction from the negative resting potential towards the positive membrane potential that will be the peak of the action potential.